{
  "term_label": "absorption of visible light",
  "gene": "UniProtKB:P08100",
  "gene_symbol": "RHO",
  "gene_name": "Rhodopsin",
  "term_id": "GO:0016038"
}